{
  "term_id": "GO:0070971",
  "gene_symbol": "CTAGE8",
  "term_label": "endoplasmic reticulum exit site",
  "gene": "UniProtKB:P0CG41",
  "gene_name": "cTAGE family member 8"
}